fatty acid primary amide biosynthetic process [GO:0062112] (biological process) Relationships: is a type of GO:0043604; is a type of fatty acid primary amide metabolic process [GO:0062126]; is a type of GO:1901570 Also known as: FAPA biosynthesis, FAPA biosynthetic process, fatty acid amide biosynthesis Definition: The chemical reactions and pathways resulting in the formation of a fatty acid primary amide. References: PMID:10079066, PMID:15952893